wall teichoic acid biosynthetic process [GO:0070398] (biological process) Also known as: WTA biosynthetic process, wall teichoic acid anabolism, wall teichoic acid biosynthesis, wall teichoic acid formation, wall teichoic acid synthesis References: PMID:14665680, PMID:16020688 Sources: GOC:add Relationships: is a type of teichoic acid biosynthetic process [GO:0019350] Definition: The chemical reactions and pathways resulting in the formation of wall teichoic acid, which is a major component of the cell wall of Gram-positive bacteria and typically consists of a polymer of glycerol-phosphate or ribitol-phosphate to which are attached glycosyl and D-alanyl ester residues and which is covalently linked to peptidoglycan.